cell adhesive protein binding involved in AV node cell-bundle of His cell communication [GO:0086082] (molecular function) Also known as: cell adhesive protein binding involved in atrioventricular node cell-bundle of His cell communication Relationships: is a type of GO:0086080; is part of AV node cell-bundle of His cell adhesion involved in cell communication [GO:0086072] Definition: Binding to a protein or protein complex that results in the connection of an AV node cell with a bundle of His cell and contributes to the communication between the two cells. Sources: GOC:BHF, GOC:mtg_cardiac_conduct_nov11